{
  "gene_symbol": "ENTPD6",
  "gene": "UniProtKB:O75354",
  "term_label": "Unknown biological process",
  "gene_name": "Ectonucleoside triphosphate diphosphohydrolase 6",
  "term_id": "UNKNOWN:0002"
}